{
  "gene_symbol": "PCNA",
  "term_id": "GO:0006298",
  "gene": "UniProtKB:P12004",
  "term_label": "mismatch repair",
  "gene_name": "Proliferating cell nuclear antigen"
}